{
  "gene": "UniProtKB:O14763",
  "gene_name": "Tumor necrosis factor receptor superfamily member 10B",
  "gene_symbol": "TNFRSF10B",
  "term_label": "cell surface",
  "term_id": "GO:0009986"
}